{
  "gene_name": "von Hippel-Lindau disease tumor suppressor",
  "gene_symbol": "VHL",
  "term_id": "UNKNOWN:0003",
  "gene": "UniProtKB:P40337",
  "term_label": "Unknown cellular component"
}